{
  "term_label": "type 1 fibroblast growth factor receptor binding",
  "gene": "UniProtKB:O76093",
  "gene_name": "Fibroblast growth factor 18",
  "gene_symbol": "FGF18",
  "term_id": "GO:0005105"
}